{
  "gene_symbol": "LGI1",
  "term_id": "GO:0005615",
  "gene": "UniProtKB:O95970",
  "gene_name": "Leucine-rich glioma-inactivated protein 1",
  "term_label": "extracellular space"
}